{
  "term_id": "UNKNOWN:0003",
  "gene_symbol": "WDR89",
  "term_label": "Unknown cellular component",
  "gene": "UniProtKB:Q96FK6",
  "gene_name": "WD repeat-containing protein 89"
}